5'-methylthioadenosine deaminase activity [GO:0090614] (molecular function) Relationships: is a type of hydrolase activity, acting on carbon-nitrogen (but not peptide) bonds, in cyclic amidines [GO:0016814]; is a type of deaminase activity [GO:0019239] References: PMID:23968233 Sources: RHEA:25025 Definition: Catalysis of the reaction: 5'methyl thioadenosine + H2O = 5'methyl thioinosine + NH3.